xenobiotic metabolic process [GO:0006805] (biological process) Definition: The chemical reactions and pathways involving a xenobiotic compound, a compound foreign to the organism exposed to it. It may be synthesized by another organism (like ampicilin) or it can be a synthetic chemical. Also known as: xenobiotic metabolism, drug metabolic process, drug metabolism Relationships: is a type of GO:0008152; is part of cellular response to xenobiotic stimulus [GO:0071466] Subtypes: insecticide metabolic process [GO:0017143], GO:0018872, cyanamide metabolic process [GO:0018890], cyclohexylsulfamate metabolic process [GO:0018892], GO:0018905, methyl tert-butyl ether metabolic process [GO:0018906], dodecyl sulfate metabolic process [GO:0018909], methanesulfonic acid metabolic process [GO:0018926], nitroglycerin metabolic process [GO:0018937], pentaerythritol tetranitrate metabolic process [GO:0018954], GO:0018964, tetrahydrofuran catabolic process [GO:0018968], GO:0018969, GO:0042178, halogenated hydrocarbon metabolic process [GO:0042197] Sources: GOC:cab2, GOC:krc